glutamate-cysteine ligase complex [GO:0017109] (cellular component) Relationships: is a type of catalytic complex [GO:1902494]; is part of GO:0005737 Also known as: gamma-glutamylcysteine synthetase complex Definition: An enzyme complex that catalyzes the ligation of glutamate to cysteine, forming glutamylcysteine. References: PMID:9675072